{
  "term_id": "UNKNOWN:0001",
  "term_label": "Unknown molecular function",
  "gene_symbol": "CCDC33",
  "gene": "UniProtKB:Q8N5R6",
  "gene_name": "Coiled-coil domain-containing protein 33"
}